{
  "term_label": "plasma membrane",
  "term_id": "GO:0005886",
  "gene_name": "GTPase-activating Rap_Ran-GAP domain-like protein 3",
  "gene_symbol": "GARNL3",
  "gene": "UniProtKB:Q5VVW2"
}